striated muscle cell proliferation [GO:0014855] (biological process) Relationships: is a type of muscle cell proliferation [GO:0033002] Definition: The multiplication or reproduction of striated muscle cells, resulting in the expansion of a cell population. Striated muscles contain fibers that are divided by transverse bands into striations, and cardiac and skeletal muscle are types of striated muscle. Sources: CL:0000737, GOC:ef, GOC:mtg_muscle Subtypes: skeletal muscle cell proliferation [GO:0014856], cardiac muscle cell proliferation [GO:0060038]